{
  "term_label": "ribonucleoprotein complex",
  "term_id": "GO:1990904",
  "gene_name": "CUGBP Elav-like family member 1",
  "gene_symbol": "CELF1",
  "gene": "UniProtKB:Q92879"
}